{
  "term_label": "Unknown biological process",
  "gene": "UniProtKB:Q2NL98",
  "gene_name": "Vimentin-type intermediate filament-associated coiled-coil protein",
  "gene_symbol": "VMAC",
  "term_id": "UNKNOWN:0002"
}